spore inner membrane [GO:0140549] (cellular component) Relationships: is a type of membrane [GO:0016020] References: PMID:23202530 Also known as: spore membrane Definition: The membrane surrounding the spore core (endospore core) that separates it from its external environment.